{
  "gene": "UniProtKB:A0A286YF58",
  "gene_name": "Transmembrane protein 271",
  "gene_symbol": "TMEM271",
  "term_id": "UNKNOWN:0001",
  "term_label": "Unknown molecular function"
}